regulation of venous endothelial cell fate commitment [GO:2000787] (biological process) Subtypes: negative regulation of venous endothelial cell fate commitment [GO:2000788], positive regulation of venous endothelial cell fate commitment [GO:2000789] References: PMID:11585794 Definition: Any process that modulates the frequency, rate or extent of venous endothelial cell fate commitment. Relationships: is a type of regulation of cell fate commitment [GO:0010453]; is a type of regulation of blood vessel endothelial cell differentiation [GO:0110057]; regulates venous endothelial cell fate commitment [GO:0060845]